{
  "gene_symbol": "DNAJC10",
  "term_id": "GO:0016671",
  "term_label": "oxidoreductase activity, acting on a sulfur group of donors, disulfide as acceptor",
  "gene": "UniProtKB:Q8IXB1",
  "gene_name": "DnaJ homolog subfamily C member 10"
}